{
  "gene_name": "SH3 and multiple ankyrin repeat domains protein 3",
  "gene": "UniProtKB:Q9BYB0",
  "term_id": "GO:0035255",
  "term_label": "ionotropic glutamate receptor binding",
  "gene_symbol": "SHANK3"
}